retina blood vessel maintenance [GO:0097601] (biological process) Relationships: is_a retina homeostasis [GO:0001895] Also known as: maintenance of retina blood vessel, maintenance of retinal blood vessel, maintenance of choriocapillaris References: PMID:23093773 Sources: GOC:jh2 Definition: A retina homeostatic process preventing the degeneration of a retina blood vessel.